L-proline biosynthetic process [GO:0055129] (biological process) Regulation: RO_0002211 by regulation of L-proline biosynthetic process [GO:1902005]; RO_0002212 by negative regulation of L-proline biosynthetic process [GO:1902006] Definition: The chemical reactions and pathways resulting in the formation of L-proline, an L-enantiomer of a chiral, cyclic, nonessential alpha-amino acid found in peptide linkage in proteins. Sources: GOC:ecd Relationships: is a type of GO:0006560; is a type of glutamine family amino acid biosynthetic process [GO:0009084] Also known as: pyrrolidine-2-carboxylic acid biosynthetic process Subtypes: GO:0019492